{
  "term_id": "GO:0005634",
  "gene_name": "Diphosphoinositol polyphosphate phosphohydrolase 3-beta",
  "gene_symbol": "NUDT11",
  "gene": "UniProtKB:Q96G61",
  "term_label": "nucleus"
}